{
  "term_label": "receptor antagonist activity",
  "gene": "UniProtKB:P0CJ77",
  "gene_symbol": "MTRNR2L10",
  "gene_name": "Humanin-like 10",
  "term_id": "GO:0048019"
}